{
  "term_label": "cysteinyl leukotriene receptor activity",
  "gene": "UniProtKB:Q9Y271",
  "gene_name": "Cysteinyl leukotriene receptor 1",
  "term_id": "GO:0001631",
  "gene_symbol": "CYSLTR1"
}